{
  "term_id": "GO:0051959",
  "term_label": "dynein light intermediate chain binding",
  "gene_symbol": "CCDC88B",
  "gene": "UniProtKB:A6NC98",
  "gene_name": "Coiled-coil domain-containing protein 88B"
}